protein-ribulosamine 3-kinase activity [GO:0102193] (molecular function) Relationships: is a type of phosphotransferase activity, alcohol group as acceptor [GO:0016773]; is a type of catalytic activity, acting on a protein [GO:0140096] Sources: EC:2.7.1.172, GOC:pz Definition: Catalysis of the reaction: ATP + a [protein]-N6-D-ribulosyl-L-lysine = ADP + a [protein]-N6-(3-O-phospho-D-ribulosyl)-L-lysine.